{
  "gene_name": "Growth_differentiation factor 7",
  "gene": "UniProtKB:Q7Z4P5",
  "term_id": "GO:0030509",
  "term_label": "BMP signaling pathway",
  "gene_symbol": "GDF7"
}